3-oxoacyl-[acyl-carrier-protein] synthase activity [GO:0004315] (molecular function) Also known as: condensing enzyme activity, fatty acid condensing enzyme activity, 3-oxoacyl-ACP synthase activity, 3-oxoacyl-[acyl-carrier protein] synthase activity, ketoacyl-ACP synthase activity, 3-oxoacyl-acyl carrier protein synthase I activity, beta-ketoacyl-ACP synthase I activity, beta-ketoacyl-ACP synthase II activity, beta-ketoacyl-acyl-carrier-protein synthase I, beta-ketoacyl-acyl-carrier-protein synthase II activity, 3-ketoacyl-acyl carrier protein synthase activity, 3-oxoacyl-acyl-carrier-protein synthase activity, acyl-acyl-carrier-protein:malonyl-acyl-carrier-protein C-acyltransferase (decarboxylating), acyl-malonyl acyl carrier protein-condensing enzyme activity, acyl-malonyl(acyl-carrier-protein)-condensing enzyme activity, beta-ketoacyl acyl carrier protein synthase activity, beta-ketoacyl synthetase activity, beta-ketoacyl-ACP synthetase activity, beta-ketoacyl-[acyl carrier protein] synthase activity, beta-ketoacyl-acyl carrier protein synthase activity, beta-ketoacyl-acyl carrier protein synthetase activity, beta-ketoacylsynthase activity Sources: RHEA:22836 Note: Note that this activity is responsible for the chain-elongation step of dissociated (type II) fatty-acid biosynthesis, i.e. the addition of two C atoms to the fatty-acid chain. Can use fatty acyl thioesters of ACP (C2 to C16) as substrates, as well as fatty acyl thioesters of Co-A (C4 to C16). Definition: Catalysis of the reaction: acyl-[acyl-carrier protein] + malonyl-[acyl-carrier protein] = 3-oxoacyl-[acyl-carrier protein] + CO2 + [acyl-carrier protein]. Relationships: is a type of acyltransferase activity, transferring groups other than amino-acyl groups [GO:0016747]